{
  "gene": "UniProtKB:O95185",
  "gene_symbol": "UNC5C",
  "term_id": "GO:0007411",
  "gene_name": "Netrin receptor UNC5C",
  "term_label": "axon guidance"
}